calcium-dependent cysteine-type endopeptidase inhibitor activity [GO:0010859] (molecular function) Definition: Binds to and stops, prevents or reduces the activity of a calcium-dependent cysteine-type endopeptidase, any enzyme that hydrolyzes peptide bonds in polypeptides by a mechanism in which the sulfhydryl group of a cysteine residue at the active center acts as a nucleophile in a calcium-dependent manner. Sources: GOC:dph, GOC:tb Relationships: is a type of GO:0004869